{
  "gene_name": "Rho GTPase-activating protein 6",
  "term_id": "GO:0015629",
  "gene_symbol": "ARHGAP6",
  "term_label": "actin cytoskeleton",
  "gene": "UniProtKB:O43182"
}